{
  "term_id": "GO:0043240",
  "gene_symbol": "CENPX",
  "gene": "UniProtKB:A8MT69",
  "gene_name": "Centromere protein X",
  "term_label": "Fanconi anaemia nuclear complex"
}